{
  "term_id": "GO:0002767",
  "gene_name": "Leukocyte immunoglobulin-like receptor subfamily A member 2",
  "term_label": "immune response-inhibiting cell surface receptor signaling pathway",
  "gene": "UniProtKB:Q8N149",
  "gene_symbol": "LILRA2"
}